transcription factor TFIIIB complex [GO:0000126] (cellular component) References: PMID:11433012 Sources: GOC:mah Definition: A transcription factor complex that is involved in regulating transcription from RNA polymerase III (Pol III) promoters. TFIIIB contains the TATA-binding protein (TBP) and two Pol III-specific proteins, B'' and BRF. Relationships: is a type of GO:0090576 Subtypes: transcription factor TFIIIB-alpha complex [GO:0034732], GO:0034733